{
  "gene_name": "Neuronal PAS domain-containing protein 2",
  "term_label": "CLOCK-BMAL transcription complex",
  "gene_symbol": "NPAS2",
  "gene": "UniProtKB:Q99743",
  "term_id": "GO:1990513"
}